{
  "gene_symbol": "STAT4",
  "term_label": "DNA-binding transcription factor activity, RNA polymerase II-specific",
  "gene_name": "Signal transducer and activator of transcription 4",
  "term_id": "GO:0000981",
  "gene": "UniProtKB:Q14765"
}